negative regulation of sphingolipid biosynthetic process [GO:0090155] (BP) Subtypes: negative regulation of ceramide biosynthetic process [GO:1900060] Relationships: is a type of negative regulation of lipid biosynthetic process [GO:0051055]; is a type of GO:0090153; negatively regulates GO:0030148 Also known as: negative regulation of sphingolipid biosynthesis involved in cellular sphingolipid homeostasis Definition: Any process that decreases the rate, frequency or extent of sphingolipid biosynthesis. Sphingolipid biosynthesis is the chemical reactions and pathways resulting in the formation of sphingolipids, any of a class of lipids containing the long-chain amine diol sphingosine or a closely related base (a sphingoid). Sources: GOC:ascb_2009, GOC:dph, GOC:tb